homologous chromosome pairing at meiosis [GO:0007129] (biological process) Definition: The meiotic cell cycle process where side by side pairing and physical juxtaposition of homologous chromosomes is created during meiotic prophase. Homologous chromosome pairing begins when the chromosome arms begin to pair from the clustered telomeres and ends when synaptonemal complex or linear element assembly is complete. References: PMID:22582262, PMID:23117617, PMID:31811152 Sources: GOC:mtg_cell_cycle Also known as: chromosomal synapsis, synapsis, chromosomal pairing Relationships: is a type of GO:0070192; is part of homologous chromosome segregation [GO:0045143]